{
  "gene_name": "Notch-regulated ankyrin repeat-containing protein",
  "gene": "UniProtKB:Q7Z6K4",
  "gene_symbol": "NRARP",
  "term_label": "negative regulation of Notch signaling pathway",
  "term_id": "GO:0045746"
}